{
  "term_id": "GO:0030247",
  "term_label": "polysaccharide binding",
  "gene_symbol": "CLEC18C",
  "gene_name": "C-type lectin domain family 18 member C",
  "gene": "UniProtKB:Q8NCF0"
}